{
  "term_label": "Unknown biological process",
  "gene": "UniProtKB:Q9NSG2",
  "term_id": "UNKNOWN:0002",
  "gene_symbol": "FIRRM",
  "gene_name": "FIGNL1-interacting regulator of recombination and mitosis"
}